{
  "gene_name": "Hydroxymethylglutaryl-CoA synthase, cytoplasmic",
  "gene_symbol": "HMGCS1",
  "gene": "UniProtKB:Q01581",
  "term_label": "farnesyl diphosphate biosynthetic process, mevalonate pathway",
  "term_id": "GO:0010142"
}